short-chain fatty acid metabolic process [GO:0046459] (biological process) Sources: Wikipedia:Fatty_acid_metabolism Also known as: short-chain fatty acid metabolism Subtypes: propionate metabolic process [GO:0019541], butyrate metabolic process [GO:0019605], short-chain fatty acid catabolic process [GO:0019626], glutamate catabolic process to 4-hydroxybutyrate [GO:0036241], acetoacetic acid metabolic process [GO:0043438], GO:0051790 Definition: The chemical reactions and pathways involving a short-chain fatty acid. A short-chain fatty acid has an aliphatic tail containing fewer than 6 carbons. Relationships: is a type of GO:0006631 Note: While there is not universal consensus on the lengths of short-, medium-, long- and very-long-chain fatty acids, the GO uses the definitions in ChEBI (see CHEBI:26666, CHEBI:59554, CHEBI:15904 and CHEBI:27283).